{
  "gene": "UniProtKB:P58170",
  "gene_symbol": "OR1D5",
  "term_id": "GO:0005886",
  "gene_name": "Olfactory receptor 1D5",
  "term_label": "plasma membrane"
}